{
  "gene_name": "Kelch-like protein 7",
  "term_label": "proteasome-mediated ubiquitin-dependent protein catabolic process",
  "gene_symbol": "KLHL7",
  "term_id": "GO:0043161",
  "gene": "UniProtKB:Q8IXQ5"
}